{
  "term_label": "histone reader activity",
  "gene_name": "Protein AF-10",
  "gene_symbol": "MLLT10",
  "gene": "UniProtKB:P55197",
  "term_id": "GO:0140566"
}